smooth muscle cell migration [GO:0014909] (biological process) Relationships: is a type of GO:0014812 Sources: CL:0000192, GOC:mtg_muscle Definition: The orderly movement of a smooth muscle cell from one site to another, often during the development of a multicellular organism. Regulation: regulated by GO:0014910; positively regulated by positive regulation of smooth muscle cell migration [GO:0014911]; negatively regulated by negative regulation of smooth muscle cell migration [GO:0014912] Subtypes: smooth muscle cell chemotaxis [GO:0071670], vascular associated smooth muscle cell migration [GO:1904738]